{
  "term_id": "GO:0004843",
  "term_label": "cysteine-type deubiquitinase activity",
  "gene": "UniProtKB:Q9UMW8",
  "gene_name": "Ubl carboxyl-terminal hydrolase 18",
  "gene_symbol": "USP18"
}